{
  "term_label": "nucleus",
  "gene_symbol": "TGS1",
  "gene": "UniProtKB:Q96RS0",
  "term_id": "GO:0005634",
  "gene_name": "Trimethylguanosine synthase"
}